{
  "gene_symbol": "ADD2",
  "term_id": "GO:0005856",
  "term_label": "cytoskeleton",
  "gene_name": "Beta-adducin",
  "gene": "UniProtKB:P35612"
}